{
  "term_label": "Unknown cellular component",
  "gene": "UniProtKB:Q9NSA0",
  "gene_symbol": "SLC22A11",
  "gene_name": "Solute carrier family 22 member 11",
  "term_id": "UNKNOWN:0003"
}